{
  "gene_name": "Receptor activity-modifying protein 3",
  "term_label": "protein transport",
  "term_id": "GO:0015031",
  "gene": "UniProtKB:O60896",
  "gene_symbol": "RAMP3"
}